{
  "gene": "UniProtKB:Q96G97",
  "gene_symbol": "BSCL2",
  "term_id": "GO:0034389",
  "term_label": "lipid droplet organization",
  "gene_name": "Seipin"
}